{
  "term_id": "GO:0005886",
  "term_label": "plasma membrane",
  "gene_name": "EH domain-containing protein 1",
  "gene_symbol": "EHD1",
  "gene": "UniProtKB:Q9H4M9"
}